{
  "term_id": "GO:0036464",
  "gene_name": "Protein argonaute-2",
  "gene_symbol": "AGO2",
  "term_label": "cytoplasmic ribonucleoprotein granule",
  "gene": "UniProtKB:Q9UKV8"
}